phenylalanine-tRNA ligase activity [GO:0004826] (molecular function) Definition: Catalysis of the reaction: ATP + L-phenylalanine + tRNA(Phe) = AMP + diphosphate + L-phenylalanyl-tRNA(Phe). Sources: EC:6.1.1.20 Also known as: phenylalanyl-tRNA synthetase activity, L-phenylalanine:tRNAPhe ligase (AMP-forming) activity, L-phenylalanyl-tRNA synthetase activity, phenylalanine translase activity, phenylalanine-tRNA synthetase activity, phenylalanyl-tRNA ligase activity, phenylalanyl-transfer RNA ligase activity, phenylalanyl-transfer RNA synthetase activity, phenylalanyl-transfer ribonucleate synthetase activity Relationships: is a type of aminoacyl-tRNA ligase activity [GO:0004812]